{
  "term_label": "respiratory burst",
  "gene_name": "Putative neutrophil cytosol factor 1B",
  "gene_symbol": "NCF1B",
  "gene": "UniProtKB:A6NI72",
  "term_id": "GO:0045730"
}